{
  "gene": "UniProtKB:O75838",
  "gene_symbol": "CIB2",
  "term_label": "magnesium ion binding",
  "gene_name": "Calcium and integrin-binding family member 2",
  "term_id": "GO:0000287"
}